cell plate [GO:0009504] (cellular component) Sources: ISBN:0198547684 Relationships: is a type of cellular anatomical structure [GO:0110165]; is part of GO:0005737 Definition: The nascent cell membrane and cell wall structure that forms between two daughter nuclei near the center of a dividing plant cell. It develops at the equatorial region of the phragmoplast. It grows outwards to join with the lateral walls and form two daughter cells.